{
  "gene_symbol": "RASGEF1A",
  "gene_name": "Ras-GEF domain-containing family member 1A",
  "term_id": "GO:0005886",
  "term_label": "plasma membrane",
  "gene": "UniProtKB:Q8N9B8"
}